tumor necrosis factor binding [GO:0043120] (MF) Relationships: is a type of GO:0019955 Definition: Binding to tumor necrosis factor, a proinflammatory cytokine produced by monocytes and macrophages. Sources: GOC:jl, http://lookwayup.com/ Subtypes: TNFSF11 binding [GO:0038057]